{
  "gene_name": "Seipin",
  "term_id": "GO:0005789",
  "gene": "UniProtKB:Q96G97",
  "gene_symbol": "BSCL2",
  "term_label": "endoplasmic reticulum membrane"
}